{
  "term_id": "GO:0004888",
  "gene_name": "CMRF35-like molecule 5",
  "gene_symbol": "CD300LD",
  "gene": "UniProtKB:Q6UXZ3",
  "term_label": "transmembrane signaling receptor activity"
}